{
  "term_id": "GO:0005178",
  "gene": "UniProtKB:P18564",
  "gene_name": "Integrin beta-6",
  "term_label": "integrin binding",
  "gene_symbol": "ITGB6"
}